{
  "gene_name": "Acetylcholine receptor subunit gamma",
  "gene": "UniProtKB:P07510",
  "term_id": "GO:0034220",
  "gene_symbol": "CHRNG",
  "term_label": "monoatomic ion transmembrane transport"
}